deoxyinosine biosynthetic process [GO:0046095] (biological process) Relationships: is a type of deoxyinosine metabolic process [GO:0046094]; is a type of purine deoxyribonucleoside biosynthetic process [GO:0046123] Subtypes: deoxyinosine salvage [GO:0006191] Definition: The chemical reactions and pathways resulting in the formation of deoxyinosine, hypoxanthine deoxyriboside. Also known as: deoxyinosine anabolism, deoxyinosine biosynthesis, deoxyinosine formation, deoxyinosine synthesis Sources: GOC:go_curators